{
  "term_id": "GO:0030687",
  "gene": "UniProtKB:Q9GZL7",
  "gene_name": "Ribosome biogenesis protein WDR12",
  "gene_symbol": "WDR12",
  "term_label": "preribosome, large subunit precursor"
}